negative regulation of luteinizing hormone secretion [GO:0033685] (biological process) Definition: Any process that stops, prevents, or reduces the frequency, rate or extent of the regulated release of luteinizing hormone. Also known as: down regulation of luteinizing hormone secretion, down-regulation of luteinizing hormone secretion, downregulation of luteinizing hormone secretion, inhibition of luteinizing hormone secretion Relationships: is a type of negative regulation of gonadotropin secretion [GO:0032277]; is a type of GO:0033684; negatively regulates GO:0032275 Sources: GOC:mah